{
  "term_label": "Unknown molecular function",
  "gene_name": "Zinc finger CCHC domain-containing protein 24",
  "gene": "UniProtKB:Q8N2G6",
  "gene_symbol": "ZCCHC24",
  "term_id": "UNKNOWN:0001"
}